response to gravity [GO:0009629] (BP) Also known as: response to gravitational stimulus Sources: GOC:hb Relationships: is a type of response to abiotic stimulus [GO:0009628] Subtypes: detection of gravity [GO:0009590], gravitropism [GO:0009630], gravitaxis [GO:0042332], cellular response to gravity [GO:0071258] Definition: Any process that results in a change in state or activity of a cell or an organism (in terms of movement, secretion, enzyme production, gene expression, etc.) as a result of a gravitational stimulus.